negative regulation of synaptic transmission, glycinergic [GO:0060093] (biological process) Definition: Any process that stops or decreases the frequency, rate or extent of glycinergic synaptic transmission. Glycinergic synaptic transmission is the process of communication from a neuron to another neuron across a synapse using the neurotransmitter glycine. Sources: GOC:dms, GOC:dph Also known as: negative regulation of glycinergic synaptic transmission Relationships: is a type of negative regulation of synaptic transmission [GO:0050805]; is a type of regulation of synaptic transmission, glycinergic [GO:0060092]; negatively regulates synaptic transmission, glycinergic [GO:0060012] Subtypes: negative regulation of glycine secretion, neurotransmission [GO:1904625]